{
  "gene_name": "Alpha-N-acetylgalactosaminidase",
  "term_label": "alpha-galactosidase activity",
  "term_id": "GO:0004557",
  "gene_symbol": "NAGA",
  "gene": "UniProtKB:P17050"
}